{
  "gene_name": "Dual specificity protein phosphatase 23",
  "term_label": "cytoplasm",
  "gene": "UniProtKB:Q9BVJ7",
  "term_id": "GO:0005737",
  "gene_symbol": "DUSP23"
}